protein-phosphocysteine-glucose phosphotransferase system transporter activity [GO:0090564] (molecular function) Definition: Catalysis of the PEP-dependent, phosphoryl transfer-driven transport of substances across a membrane. The transport happens by catalysis of the reaction: protein S-phosphocysteine + glucose(out) = protein cysteine + glucose phosphate(in). This differs from primary and secondary active transport in that the solute is modified during transport. Relationships: is_a protein-phosphocysteine-sugar phosphotransferase activity [GO:0090563] Sources: GOC:am